{
  "term_id": "GO:0005886",
  "gene": "UniProtKB:Q9Y5N1",
  "gene_name": "Histamine H3 receptor",
  "term_label": "plasma membrane",
  "gene_symbol": "HRH3"
}